positive regulation of nucleoside metabolic process [GO:0045979] (biological process) Relationships: is a type of GO:0009118; is a type of GO:0062013; positively regulates nucleoside metabolic process [GO:0009116] Sources: GOC:go_curators Definition: Any process that activates or increases the frequency, rate or extent of the chemical reactions and pathways involving nucleosides. Also known as: positive regulation of nucleoside metabolism, up regulation of nucleoside metabolic process, up-regulation of nucleoside metabolic process, upregulation of nucleoside metabolic process, activation of nucleoside metabolic process, stimulation of nucleoside metabolic process